licheninase activity [GO:0042972] (molecular function) Definition: Catalysis of the hydrolysis of (1->4)-beta-D-glucosidic linkages in beta-D-glucans containing (1->3) and (1->4) bonds. Sources: EC:3.2.1.73 Also known as: beta-glucanase activity, 1,3-1,4-beta-D-glucan 4-glucanohydrolase activity, 1,3-1,4-beta-glucan 4-glucanohydrolase activity, lichenase activity, 1,3;1,4-beta-glucan 4-glucanohydrolase activity, 1,3;1,4-beta-glucan endohydrolase activity, beta-(1->3), (1->4)-D-glucan 4-glucanohydrolase activity, endo-beta-1,3-1,4 glucanase activity, mixed linkage beta-glucanase activity Relationships: is a type of GO:0004553